regulation of meiotic joint molecule formation [GO:0010946] (biological process) Relationships: is_a regulation of cell cycle process [GO:0010564]; is a type of GO:2000241; regulates GO:0000709 Definition: Any process that modulates the frequency, rate or extent of meiotic joint molecule formation. Meiotic joint molecule formation is the conversion of the paired broken DNA and homologous duplex DNA into a four-stranded branched intermediate, known as a joint molecule, formed during meiotic recombination. Sources: GOC:dph, GOC:tb Subtypes: negative regulation of meiotic joint molecule formation [GO:0010947]